{
  "term_label": "regulation of cytokine production",
  "gene_symbol": "ZBTB33",
  "gene_name": "Transcriptional regulator Kaiso",
  "gene": "UniProtKB:Q86T24",
  "term_id": "GO:0001817"
}